mitochondrial respiratory chain complex assembly [GO:0033108] (biological process) Relationships: is_a protein-containing complex assembly [GO:0065003]; is part of mitochondrion organization [GO:0007005]; occurs in mitochondrion [GO:0005739] Subtypes: GO:0032981, mitochondrial proton-transporting ATP synthase complex assembly [GO:0033615], mitochondrial respiratory chain complex IV assembly [GO:0033617], mitochondrial respiratory chain complex III assembly [GO:0034551], mitochondrial respiratory chain complex II assembly [GO:0034553], mitochondrial respirasome assembly [GO:0097250] Sources: GOC:mah Definition: The aggregation, arrangement and bonding together of a set of components to form a mitochondrial respiratory chain complex or between respiratory chain complexes to form high-order structures.